{
  "term_label": "Unknown biological process",
  "gene_name": "Cilia- and flagella-associated protein 141",
  "term_id": "UNKNOWN:0002",
  "gene": "UniProtKB:Q5VU69",
  "gene_symbol": "CFAP141"
}